toluene oxidation via 2-hydroxytoluene [GO:0019601] (biological process) Definition: The degradation of toluene to form pyruvate and acetaldehyde; the first step in the pathway is the oxidation of toluene to form 2-hydroxytoluene (o-cresol). Relationships: is a type of GO:0019600 Sources: MetaCyc:TOLUENE-DEG-2-OH-PWY